{
  "term_label": "Unknown biological process",
  "gene": "UniProtKB:P21796",
  "gene_symbol": "VDAC1",
  "term_id": "UNKNOWN:0002",
  "gene_name": "Voltage-dependent anion-selective channel protein 1"
}